{
  "term_label": "ribonuclease H2 complex",
  "gene_name": "Ribonuclease H2 subunit A",
  "gene": "UniProtKB:O75792",
  "gene_symbol": "RNASEH2A",
  "term_id": "GO:0032299"
}